choline biosynthetic process via N-monomethylethanolamine [GO:0033324] (biological process) Also known as: choline anabolism via N-monomethylethanolamine, choline biosynthesis via N-monomethylethanolamine, choline formation via N-monomethylethanolamine, choline synthesis via N-monomethylethanolamine Definition: The chemical reactions and pathways resulting in the formation of choline (2-hydroxyethyltrimethylammonium), via the intermediate N-monomethylethanolamine. Relationships: is a type of choline biosynthetic process [GO:0042425] Sources: GOC:mah, MetaCyc:PWY-3542